myotube cell development involved in skeletal muscle regeneration [GO:0014906] (biological process) Sources: GOC:mtg_muscle Definition: The process aimed at the progression of a myotube cell over time, from initial commitment of the cell to a specific fate, to the fully functional differentiated cell. This occurs as part of the process of skeletal muscle regeneration. Myotubes are multinucleated cells that are formed when proliferating myoblasts exit the cell cycle, differentiate and fuse. Relationships: is a type of myotube cell development [GO:0014904]; is part of myotube differentiation involved in skeletal muscle regeneration [GO:0014908]